{
  "gene_name": "ABI gene family member 3",
  "term_id": "GO:0030027",
  "gene": "UniProtKB:Q9P2A4",
  "term_label": "lamellipodium",
  "gene_symbol": "ABI3"
}